{
  "term_id": "GO:0031295",
  "gene_symbol": "TNFRSF13C",
  "term_label": "T cell costimulation",
  "gene_name": "Tumor necrosis factor receptor superfamily member 13C",
  "gene": "UniProtKB:Q96RJ3"
}